{
  "gene_symbol": "COQ5",
  "term_id": "GO:0008425",
  "gene_name": "2-methoxy-6-polyprenyl-1,4-benzoquinol methylase, mitochondrial",
  "gene": "UniProtKB:Q5HYK3",
  "term_label": "2-methoxy-6-polyprenyl-1,4-benzoquinol methyltransferase activity"
}